valine dehydrogenase (NADP+) activity [GO:0050391] (molecular function) Sources: EC:1.4.1.8, MetaCyc:VALINE-DEHYDROGENASE-NADP+-RXN Relationships: is a type of oxidoreductase activity, acting on the CH-NH2 group of donors, NAD or NADP as acceptor [GO:0016639] Also known as: valine dehydrogenase (NADP) activity, L-valine:NADP+ oxidoreductase (deaminating), valine dehydrogenase (nicotinanide adenine dinucleotide phosphate) Definition: Catalysis of the reaction: L-valine + H2O + NADP+ = 3-methyl-2-oxobutanoate + NH3 + NADPH.